{
  "gene": "UniProtKB:O15066",
  "term_label": "microtubule-based movement",
  "term_id": "GO:0007018",
  "gene_name": "Kinesin-like protein KIF3B",
  "gene_symbol": "KIF3B"
}